{
  "gene_symbol": "MBD4",
  "gene": "UniProtKB:O95243",
  "term_label": "DNA binding",
  "gene_name": "Methyl-CpG-binding domain protein 4",
  "term_id": "GO:0003677"
}